somatic diversification of immune receptors by N region addition [GO:0002569] (BP) Subtypes: somatic diversification of immunoglobulin genes by N region addition [GO:0002570], somatic diversification of T cell receptor genes by N region addition [GO:0002571] Definition: The addition of variable numbers of random nucleotides by terminal deoxytransferase in the N regions of heavy chain immunoglobulin and T cell receptor genes. N regions are found at the V-D, D-D, V-J, and D-J recombinational junctions, depending on the immune receptor gene. Relationships: is_a GO:0002200 Sources: GOC:add, ISBN:0781735149